{
  "term_label": "nucleus",
  "gene": "UniProtKB:A6NJZ7",
  "gene_symbol": "RIMBP3C",
  "term_id": "GO:0005634",
  "gene_name": "RIMS-binding protein 3C"
}